{
  "term_label": "RNA polymerase II cis-regulatory region sequence-specific DNA binding",
  "gene": "UniProtKB:P36508",
  "gene_symbol": "ZNF76",
  "gene_name": "Zinc finger protein 76",
  "term_id": "GO:0000978"
}